{
  "gene": "UniProtKB:Q13563",
  "term_id": "GO:0005267",
  "gene_name": "Polycystin-2",
  "gene_symbol": "PKD2",
  "term_label": "potassium channel activity"
}